{
  "gene_name": "Solute carrier family 53 member 1",
  "term_label": "phosphate transmembrane transporter activity",
  "term_id": "GO:0005315",
  "gene_symbol": "XPR1",
  "gene": "UniProtKB:Q9UBH6"
}